{
  "gene_symbol": "NOTCH2",
  "term_id": "GO:0005886",
  "gene_name": "Neurogenic locus notch homolog protein 2",
  "term_label": "plasma membrane",
  "gene": "UniProtKB:Q04721"
}